{
  "gene": "UniProtKB:Q9BSK0",
  "gene_name": "MARVEL domain-containing protein 1",
  "term_id": "GO:0019911",
  "gene_symbol": "MARVELD1",
  "term_label": "structural constituent of myelin sheath"
}